striated muscle myosin thick filament assembly [GO:0071688] (biological process) Definition: The aggregation, arrangement and bonding together of proteins to form the myosin-based thick filaments of myofibrils in striated muscle. Sources: GOC:mah Relationships: is a type of cellular component assembly involved in morphogenesis [GO:0010927]; is_a myosin filament assembly [GO:0031034]; is part of myofibril assembly [GO:0030239] Subtypes: skeletal muscle myosin thick filament assembly [GO:0030241], cardiac muscle myosin thick filament assembly [GO:0071690]